{
  "gene": "UniProtKB:Q8N109",
  "gene_symbol": "KIR2DL5A",
  "gene_name": "Killer cell immunoglobulin-like receptor 2DL5A",
  "term_id": "GO:0140375",
  "term_label": "immune receptor activity"
}